protein N-linked glycosylation via asparagine [GO:0018279] (biological process) Also known as: protein amino acid N-linked glycosylation via asparagine Sources: GOC:jsg Relationships: is a type of GO:0006487 Definition: The glycosylation of protein via the N4 atom of peptidyl-asparagine forming N4-glycosyl-L-asparagine; the most common form is N-acetylglucosaminyl asparagine; N-acetylgalactosaminyl asparagine and N4 glucosyl asparagine also occur. This modification typically occurs in extracellular peptides with an N-X-(ST) motif. Partial modification has been observed to occur with cysteine, rather than serine or threonine, in the third position; secondary structure features are important, and proline in the second or fourth positions inhibits modification.